{
  "term_label": "cytoskeleton",
  "gene_name": "Keratin, type I cytoskeletal 24",
  "gene": "UniProtKB:Q2M2I5",
  "term_id": "GO:0005856",
  "gene_symbol": "KRT24"
}